MTREC complex [GO:1990477] (cellular component) Relationships: is a type of nuclear protein-containing complex [GO:0140513] Definition: Protein complex formed by an RNA binding protein Red1, an RNA helicase Mtl1, Red5, Rmn1, Iss10/Pir1, and Ars2/Pir2. This complex is required for the recruitment of the nuclear exosome to Mmi1 nuclear focus. It is likely related to the human CBCN complex. This complex is also known as RNA silencing (NURS) complex. References: PMID:24210919, PMID:24713849, PMID:32012158 Also known as: Mtl1-Red1 core complex, NURS complex, PAXT complex